{
  "term_id": "UNKNOWN:0002",
  "gene_symbol": "FAM78A",
  "gene_name": "Protein FAM78A",
  "gene": "UniProtKB:Q5JUQ0",
  "term_label": "Unknown biological process"
}